negative regulation of synapse organization [GO:1905809] (biological process) Definition: Any process that stops, prevents or reduces the frequency, rate or extent of synapse organization. Relationships: is a type of regulation of synapse organization [GO:0050807]; is a type of GO:0051129; negatively regulates synapse organization [GO:0050808] References: PMID:27779093 Sources: GOC:TermGenie, GO_REF:0000058 Also known as: down regulation of synapse development, down regulation of synapse organisation, down regulation of synapse organization, down-regulation of synapse development, down-regulation of synapse organisation, down-regulation of synapse organization, downregulation of synapse development, downregulation of synapse organisation, downregulation of synapse organization, negative regulation of synapse development, negative regulation of synapse organisation, inhibition of synapse development, inhibition of synapse organisation, inhibition of synapse organization, down regulation of synapse morphogenesis, down regulation of synapse organization and biogenesis, down-regulation of synapse morphogenesis, down-regulation of synapse organization and biogenesis, downregulation of synapse morphogenesis, downregulation of synapse organization and biogenesis, inhibition of synapse morphogenesis, inhibition of synapse organization and biogenesis, negative regulation of synapse morphogenesis, negative regulation of synapse organization and biogenesis Subtypes: negative regulation of synapse assembly [GO:0051964], negative regulation of postsynaptic membrane organization [GO:1901627], negative regulation of presynaptic membrane organization [GO:1901630], negative regulation of neuromuscular junction development [GO:1904397], negative regulation of synapse pruning [GO:1905807], negative regulation of synapse maturation [GO:2000297]